{
  "gene_name": "Homeobox protein Hox-B8",
  "gene": "UniProtKB:P17481",
  "term_id": "GO:0000981",
  "term_label": "DNA-binding transcription factor activity, RNA polymerase II-specific",
  "gene_symbol": "HOXB8"
}